{
  "gene": "UniProtKB:Q9NTX7",
  "term_label": "ubiquitin-protein transferase activity",
  "gene_name": "E3 ubiquitin-protein ligase RNF146",
  "term_id": "GO:0004842",
  "gene_symbol": "RNF146"
}